{
  "gene": "UniProtKB:Q9NPA1",
  "term_label": "voltage-gated potassium channel complex",
  "term_id": "GO:0008076",
  "gene_symbol": "KCNMB3",
  "gene_name": "Calcium-activated potassium channel subunit beta-3"
}